heparan sulfate proteoglycan metabolic process [GO:0030201] (biological process) Also known as: heparan sulfate proteoglycan metabolism, heparan sulphate proteoglycan metabolic process, heparan sulphate proteoglycan metabolism, heparin proteoglycan metabolic process Subtypes: heparan sulfate proteoglycan biosynthetic process [GO:0015012], heparan sulfate proteoglycan catabolic process [GO:0030200] Definition: The chemical reactions and pathways involving heparan sulfate proteoglycans, which consist of a core protein linked to a heparan sulfate glycosaminoglycan. The heparan sulfate chain is composed of the repeating disaccharide unit beta-(1,4)-N-acetyl-D-glucosamine-alpha-(1,4)-hexuronic acid, the former being either sulfated or deacetylated on its amino group as well as sulfated on one of its hydroxyl groups, and the latter being a mixture of sulfated and nonsulfated D-glucuronic and L-iduronic acids. Relationships: is a type of proteoglycan metabolic process [GO:0006029] References: PMID:27241222